cytoplasmic side of plasma membrane, cell tip [GO:0106186] (cellular component) Definition: The leaflet the plasma membrane at the cell tip that faces the cytoplasm and any proteins embedded or anchored in it or attached to its surface. References: PMID:28292899 Sources: GOC:vw Relationships: is a type of GO:0009898; is part of plasma membrane of cell tip [GO:0031520]